{
  "gene_name": "DNA dC-dU-editing enzyme APOBEC-3G",
  "term_label": "P-body",
  "gene": "UniProtKB:Q9HC16",
  "gene_symbol": "APOBEC3G",
  "term_id": "GO:0000932"
}